{
  "gene_name": "Serine_threonine-protein kinase mTOR",
  "term_label": "TORC1 complex",
  "term_id": "GO:0031931",
  "gene_symbol": "MTOR",
  "gene": "UniProtKB:P42345"
}